{
  "gene_symbol": "LDLRAD3",
  "gene_name": "Low-density lipoprotein receptor class A domain-containing protein 3",
  "term_id": "GO:0005886",
  "gene": "UniProtKB:Q86YD5",
  "term_label": "plasma membrane"
}